{
  "term_id": "GO:0044331",
  "gene": "UniProtKB:Q9NYQ6",
  "term_label": "cell-cell adhesion mediated by cadherin",
  "gene_symbol": "CELSR1",
  "gene_name": "Cadherin EGF LAG seven-pass G-type receptor 1"
}